{
  "term_label": "axon guidance receptor activity",
  "gene": "UniProtKB:Q13308",
  "gene_symbol": "PTK7",
  "term_id": "GO:0008046",
  "gene_name": "Inactive tyrosine-protein kinase 7"
}